{
  "term_id": "GO:0010360",
  "gene": "UniProtKB:A6NFQ2",
  "gene_name": "TRPM8 channel-associated factor 2",
  "term_label": "negative regulation of anion channel activity",
  "gene_symbol": "TCAF2"
}